21-deoxycortisol binding [GO:1903877] (molecular function) References: PMID:10802282 Sources: GOC:TermGenie, GOC:mr, GO_REF:0000067 Definition: Binding to 21-deoxycortisol. Relationships: is a type of steroid binding [GO:0005496]; is a type of alcohol binding [GO:0043178]